{
  "gene_name": "Transmembrane protein 254",
  "gene_symbol": "TMEM254",
  "term_label": "Unknown biological process",
  "gene": "UniProtKB:Q8TBM7",
  "term_id": "UNKNOWN:0002"
}